{
  "gene_name": "Protein unc-13 homolog C",
  "term_id": "GO:0016082",
  "gene": "UniProtKB:Q8NB66",
  "term_label": "synaptic vesicle priming",
  "gene_symbol": "UNC13C"
}